{
  "gene_symbol": "LOXL4",
  "gene_name": "Lysyl oxidase homolog 4",
  "gene": "UniProtKB:Q96JB6",
  "term_label": "collagen fibril organization",
  "term_id": "GO:0030199"
}